protein binding involved in heterotypic cell-cell adhesion [GO:0086080] (molecular function) Definition: Binding to a protein or protein complex contributing to the adhesion of two different types of cells. Sources: GOC:BHF, GOC:mtg_cardiac_conduct_nov11 Relationships: is a type of cell-cell adhesion mediator activity [GO:0098632]; is part of heterotypic cell-cell adhesion [GO:0034113] Subtypes: cell adhesive protein binding involved in atrial cardiac muscle cell-AV node cell communication [GO:0086081], cell adhesive protein binding involved in AV node cell-bundle of His cell communication [GO:0086082], GO:0086083, cell adhesive protein binding involved in Purkinje myocyte-ventricular cardiac muscle cell communication [GO:0086084], cell adhesive protein binding involved in SA cardiac muscle cell-atrial cardiac muscle cell communication [GO:0086085]